{
  "gene": "UniProtKB:Q8IYN6",
  "gene_symbol": "UBALD2",
  "gene_name": "UBA-like domain-containing protein 2",
  "term_id": "UNKNOWN:0003",
  "term_label": "Unknown cellular component"
}